pleated septate junction [GO:0005919] (cellular component) Definition: A septate junction in which regular arrays of electron-dense septae span the intermembrane space. Also known as: pleated desmosome References: PMID:11700298 Relationships: is a type of septate junction [GO:0005918]